{
  "gene": "UniProtKB:Q9H1H9",
  "gene_name": "Kinesin-like protein KIF13A",
  "gene_symbol": "KIF13A",
  "term_id": "GO:0005871",
  "term_label": "kinesin complex"
}